{
  "gene_name": "Homeobox protein Hox-A13",
  "gene_symbol": "HOXA13",
  "term_id": "GO:0006357",
  "gene": "UniProtKB:P31271",
  "term_label": "regulation of transcription by RNA polymerase II"
}